{
  "gene": "UniProtKB:P19113",
  "gene_symbol": "HDC",
  "gene_name": "Histidine decarboxylase",
  "term_id": "GO:0004398",
  "term_label": "histidine decarboxylase activity"
}